{
  "gene": "UniProtKB:Q14694",
  "gene_symbol": "USP10",
  "term_label": "DNA damage response, signal transduction by p53 class mediator",
  "gene_name": "Ubiquitin carboxyl-terminal hydrolase 10",
  "term_id": "GO:0030330"
}